{
  "term_id": "GO:0000030",
  "gene_name": "Protein O-mannosyl-transferase TMTC4",
  "gene": "UniProtKB:Q5T4D3",
  "gene_symbol": "TMTC4",
  "term_label": "mannosyltransferase activity"
}